{
  "gene_symbol": "B2M",
  "gene_name": "Beta-2-microglobulin",
  "term_label": "peptide antigen binding",
  "term_id": "GO:0042605",
  "gene": "UniProtKB:P61769"
}